{
  "term_label": "Unknown cellular component",
  "term_id": "UNKNOWN:0003",
  "gene": "UniProtKB:A0A1B0GVZ9",
  "gene_symbol": "TMEM269",
  "gene_name": "Transmembrane protein 269"
}